{
  "term_id": "GO:0000981",
  "gene": "UniProtKB:Q12837",
  "gene_symbol": "POU4F2",
  "gene_name": "POU domain, class 4, transcription factor 2",
  "term_label": "DNA-binding transcription factor activity, RNA polymerase II-specific"
}